{
  "term_id": "GO:0005096",
  "gene_symbol": "ARFGAP3",
  "gene_name": "ADP-ribosylation factor GTPase-activating protein 3",
  "gene": "UniProtKB:Q9NP61",
  "term_label": "GTPase activator activity"
}